{
  "gene_name": "Keratin, type II cytoskeletal 71",
  "gene_symbol": "KRT71",
  "term_id": "GO:0030280",
  "gene": "UniProtKB:Q3SY84",
  "term_label": "structural constituent of skin epidermis"
}